{
  "term_id": "GO:0005634",
  "gene_name": "Cysteine and glycine-rich protein 2",
  "gene": "UniProtKB:Q16527",
  "gene_symbol": "CSRP2",
  "term_label": "nucleus"
}